{
  "term_label": "cell differentiation",
  "term_id": "GO:0030154",
  "gene_name": "Nuclear receptor subfamily 1 group I member 3",
  "gene_symbol": "NR1I3",
  "gene": "UniProtKB:Q14994"
}